{
  "gene_symbol": "CLEC2A",
  "term_id": "GO:0046703",
  "term_label": "natural killer cell lectin-like receptor binding",
  "gene": "UniProtKB:Q6UVW9",
  "gene_name": "C-type lectin domain family 2 member A"
}